{
  "gene": "UniProtKB:Q9HB96",
  "gene_name": "Fanconi anemia group E protein",
  "gene_symbol": "FANCE",
  "term_label": "Fanconi anaemia nuclear complex",
  "term_id": "GO:0043240"
}